{
  "term_label": "extracellular space",
  "gene_name": "C-X-C motif chemokine 16",
  "gene_symbol": "CXCL16",
  "gene": "UniProtKB:Q9H2A7",
  "term_id": "GO:0005615"
}